{
  "term_id": "GO:0008305",
  "gene_name": "Integrin beta-4",
  "term_label": "integrin complex",
  "gene_symbol": "ITGB4",
  "gene": "UniProtKB:P16144"
}